{
  "gene_symbol": "DMKN",
  "term_label": "Unknown molecular function",
  "gene_name": "Dermokine",
  "term_id": "UNKNOWN:0001",
  "gene": "UniProtKB:Q6E0U4"
}